negative regulation of striated muscle contraction [GO:0045988] (biological process) Definition: Any process that stops, prevents, or reduces the frequency, rate or extent of striated muscle contraction. Sources: GOC:go_curators Also known as: down regulation of striated muscle contraction, down-regulation of striated muscle contraction, downregulation of striated muscle contraction, inhibition of striated muscle contraction Relationships: is a type of regulation of striated muscle contraction [GO:0006942]; is a type of GO:0045932; negatively regulates striated muscle contraction [GO:0006941] Subtypes: GO:0014748, negative regulation of skeletal muscle contraction by regulation of release of sequestered calcium ion [GO:0014811], negative regulation of fast-twitch skeletal muscle fiber contraction [GO:0031447], negative regulation of slow-twitch skeletal muscle fiber contraction [GO:0031450], negative regulation of cardiac muscle contraction [GO:0055118]